{
  "gene_symbol": "FAF2",
  "term_id": "GO:0005783",
  "gene": "UniProtKB:Q96CS3",
  "term_label": "endoplasmic reticulum",
  "gene_name": "FAS-associated factor 2"
}